{
  "gene_symbol": "PCDH10",
  "term_id": "GO:0050839",
  "term_label": "cell adhesion molecule binding",
  "gene": "UniProtKB:Q9P2E7",
  "gene_name": "Protocadherin-10"
}